{
  "gene_name": "Multiple epidermal growth factor-like domains protein 9",
  "gene_symbol": "MEGF9",
  "term_id": "UNKNOWN:0003",
  "term_label": "Unknown cellular component",
  "gene": "UniProtKB:Q9H1U4"
}